{
  "gene_symbol": "CAPN5",
  "gene": "UniProtKB:O15484",
  "gene_name": "Calpain-5",
  "term_id": "GO:0004198",
  "term_label": "calcium-dependent cysteine-type endopeptidase activity"
}